{
  "gene_name": "Eyes absent homolog 1",
  "term_id": "GO:0045739",
  "gene": "UniProtKB:Q99502",
  "gene_symbol": "EYA1",
  "term_label": "positive regulation of DNA repair"
}